{
  "gene_name": "Leucine zipper putative tumor suppressor 1",
  "term_label": "Unknown molecular function",
  "gene_symbol": "LZTS1",
  "gene": "UniProtKB:Q9Y250",
  "term_id": "UNKNOWN:0001"
}